{
  "gene_symbol": "HIPK1",
  "gene": "UniProtKB:Q86Z02",
  "gene_name": "Homeodomain-interacting protein kinase 1",
  "term_id": "GO:0004674",
  "term_label": "protein serine/threonine kinase activity"
}